mitotic pre-replicative complex assembly [GO:1902985] (biological process) Relationships: is a type of GO:0006267; is a type of mitotic cell cycle process [GO:1903047]; is part of mitotic DNA replication [GO:1902969] Sources: GOC:TermGenie, GO_REF:0000060 Also known as: nuclear pre-replicative complex assembly involved in mitotic cell cycle, pre-replicative complex assembly involved in mitotic cell cycle DNA replication Definition: Any pre-replicative complex assembly involved in mitotic cell cycle DNA replication.